granzyme-mediated programmed cell death signaling pathway [GO:0140507] (BP) Definition: The series of molecular signals induced by granzymes which triggers the cell death of a cell. The pathway starts with reception of a granzyme signal, and ends when the execution phase of cell death is triggered. Granzymes are serine proteases that are secreted by cytotoxic T cells and natural killer cells to induce cell death in target cells. Also known as: granzyme-mediated cell death signaling pathway Relationships: is a type of GO:0007165; is part of programmed cell death [GO:0012501] References: PMID:32299851 Subtypes: granzyme-mediated apoptotic signaling pathway [GO:0008626]